sarcoplasm [GO:0016528] (cellular component) Sources: ISBN:0198547684 Definition: The cytoplasm of a muscle cell; includes the sarcoplasmic reticulum. Relationships: is a type of cytoplasm [GO:0005737]